{
  "gene": "UniProtKB:P0DMC3",
  "gene_name": "Apelin receptor early endogenous ligand",
  "term_id": "GO:0005179",
  "gene_symbol": "APELA",
  "term_label": "hormone activity"
}